ATPase-coupled arsenite transmembrane transporter activity [GO:0015446] (molecular function) Also known as: arsenite transporting ATPase activity, arsenite ABC transporter, arsenical pump-driving ATPase activity, arsenical resistance ATPase activity, arsenical resistance efflux pump, arsenite-translocating ATPase activity, arsenite-transmembrane transporting ATPase activity, arsenite-transporting ATPase activity Note: EC:7.3.2.7 states that this bacterial transporter does not belong to the ABC superfamily, and instead is a member of its own family, referred to as the Ars family. Like ABC transporters, it contains two nucleotide binding sites (PMID:10970874). Relationships: is a type of ATPase-coupled transmembrane transporter activity [GO:0042626]; is a type of arsenate ion transmembrane transporter activity [GO:1901683]; is part of GO:0071722 Definition: Enables the transfer of a solute or solutes from one side of a membrane to the other according to the reaction: ATP + H2O + arsenite(in) = ADP + phosphate + arsenite(out). References: PMID:10970874 Sources: RHEA:11348